{
  "gene_symbol": "IFNB1",
  "gene_name": "Interferon beta",
  "term_id": "GO:0005125",
  "term_label": "cytokine activity",
  "gene": "UniProtKB:P01574"
}